{
  "term_label": "Unknown biological process",
  "gene_symbol": "TNFRSF10D",
  "gene_name": "Tumor necrosis factor receptor superfamily member 10D",
  "term_id": "UNKNOWN:0002",
  "gene": "UniProtKB:Q9UBN6"
}